{
  "gene_name": "Acetyl-CoA acetyltransferase, cytosolic",
  "gene_symbol": "ACAT2",
  "gene": "UniProtKB:Q9BWD1",
  "term_id": "GO:0003985",
  "term_label": "acetyl-CoA C-acetyltransferase activity"
}